{
  "gene": "UniProtKB:Q9H501",
  "term_label": "RNA binding",
  "term_id": "GO:0003723",
  "gene_name": "ESF1 homolog",
  "gene_symbol": "ESF1"
}